{
  "term_id": "GO:2000779",
  "term_label": "regulation of double-strand break repair",
  "gene_symbol": "PPP4R3B",
  "gene": "UniProtKB:Q5MIZ7",
  "gene_name": "Serine_threonine-protein phosphatase 4 regulatory subunit 3B"
}